{
  "term_id": "GO:0004602",
  "gene_name": "Glutathione S-transferase 3, mitochondrial",
  "gene_symbol": "MGST3",
  "term_label": "glutathione peroxidase activity",
  "gene": "UniProtKB:O14880"
}